toluene oxidation via toluene-cis-1,2-dihydrodiol [GO:0019696] (biological process) Definition: The degradation of toluene to form pyruvate and acetaldehyde; the first step in the pathway is the oxidation of toluene to form toluene-cis-1,2-dihydrodiol. Sources: MetaCyc:TOLUENE-DEG-DIOL-PWY Relationships: is a type of GO:0019600